{
  "term_id": "GO:0043005",
  "term_label": "neuron projection",
  "gene_name": "Type II inositol 1,4,5-trisphosphate 5-phosphatase",
  "gene": "UniProtKB:P32019",
  "gene_symbol": "INPP5B"
}